Cbp3p-Cbp6 complex [GO:0061671] (cellular component) References: PMID:21670217 Sources: GOC:dph, GOC:rb Definition: A protein complex located at the mitochondrial ribosome tunnel exit that is involved in efficient translation and protein complex assembly. Relationships: is a type of mitochondrial protein-containing complex [GO:0098798]